{
  "gene_name": "Beta-3 adrenergic receptor",
  "gene": "UniProtKB:P13945",
  "gene_symbol": "ADRB3",
  "term_id": "GO:0051379",
  "term_label": "epinephrine binding"
}